{
  "term_id": "GO:0000977",
  "gene_symbol": "LHX5",
  "term_label": "RNA polymerase II transcription regulatory region sequence-specific DNA binding",
  "gene_name": "LIM_homeobox protein Lhx5",
  "gene": "UniProtKB:Q9H2C1"
}